{
  "gene_name": "Tubulin beta-3 chain",
  "term_id": "GO:0000226",
  "gene": "UniProtKB:Q13509",
  "gene_symbol": "TUBB3",
  "term_label": "microtubule cytoskeleton organization"
}